{
  "term_id": "GO:0003723",
  "term_label": "RNA binding",
  "gene_name": "Protein RRP5 homolog",
  "gene": "UniProtKB:Q14690",
  "gene_symbol": "PDCD11"
}